deoxynucleotide transmembrane transporter activity [GO:0030233] (molecular function) References: PMID:11226231 Relationships: is a type of nucleotide transmembrane transporter activity [GO:0015215]; is part of deoxynucleotide transport [GO:0030302] Definition: Catalyzes transport of all four deoxy (d) NDPs, and, less efficiently, the corresponding dNTPs, in exchange for dNDPs, ADP, or ATP.